{
  "term_id": "GO:0001965",
  "gene_name": "Synembryn-B",
  "term_label": "G-protein alpha-subunit binding",
  "gene_symbol": "RIC8B",
  "gene": "UniProtKB:Q9NVN3"
}